{
  "gene_name": "Testis-specific protein 10-interacting protein",
  "gene_symbol": "TSGA10IP",
  "term_id": "GO:0044782",
  "gene": "UniProtKB:Q3SY00",
  "term_label": "cilium organization"
}